{
  "gene_symbol": "MYO1D",
  "term_label": "microvillus",
  "gene_name": "Unconventional myosin-Id",
  "gene": "UniProtKB:O94832",
  "term_id": "GO:0005902"
}